{
  "gene_name": "Interleukin-1 receptor-associated kinase 3",
  "gene_symbol": "IRAK3",
  "gene": "UniProtKB:Q9Y616",
  "term_id": "GO:0035556",
  "term_label": "intracellular signal transduction"
}